{
  "gene": "UniProtKB:P42127",
  "term_id": "GO:0032438",
  "gene_name": "Agouti-signaling protein",
  "term_label": "melanosome organization",
  "gene_symbol": "ASIP"
}